{
  "gene_name": "Cyclin-A2",
  "gene_symbol": "CCNA2",
  "term_id": "GO:0005737",
  "term_label": "cytoplasm",
  "gene": "UniProtKB:P20248"
}